[acyl-carrier-protein] S-malonyltransferase activity [GO:0004314] (molecular function) Relationships: is a type of GO:0016419 Also known as: malonyl transacylase activity, malonyl transferase activity, ACP S-malonyltransferase activity, [acyl-carrier protein] S-malonyltransferase activity, FabD, MAT, MCAT activity, acyl carrier protein malonyltransferase activity, acyl carrier proteinmalonyltransferase activity, acyl-carrier-protein S-malonyltransferase activity, malonyl coenzyme A-acyl carrier protein transacylase activity, malonyl-CoA-acyl carrier protein transacylase activity, malonyl-CoA:ACP transacylase activity, malonyl-CoA:AcpM transacylase activity, malonyl-CoA:acyl carrier protein transacylase activity, malonyl-CoA:acyl-carrier-protein S-malonyltransferase activity Sources: EC:2.3.1.39 Definition: Catalysis of the reaction: malonyl-CoA + [acyl-carrier protein] = CoA + malonyl-[acyl-carrier protein].